DNA replication-dependent chromatin disassembly [GO:0140889] (biological process) Relationships: is a type of chromatin organization [GO:0006325] Definition: The disruption of nucleosomes during DNA replication to allow the replication machinery to access the DNA. References: PMID:34471130, PMID:35308047